{
  "gene": "UniProtKB:Q5VSD8",
  "gene_symbol": "Q5VSD8",
  "gene_name": "Putative uncharacterized protein LOC401522",
  "term_id": "UNKNOWN:0001",
  "term_label": "Unknown molecular function"
}